{
  "gene_name": "Putative uncharacterized protein KIF25-AS1",
  "term_label": "Unknown molecular function",
  "term_id": "UNKNOWN:0001",
  "gene": "UniProtKB:Q9Y6Z4",
  "gene_symbol": "KIF25-AS1"
}